{
  "gene_symbol": "RNF152",
  "term_label": "negative regulation of TORC1 signaling",
  "term_id": "GO:1904262",
  "gene": "UniProtKB:Q8N8N0",
  "gene_name": "E3 ubiquitin-protein ligase RNF152"
}